{
  "term_id": "GO:0008270",
  "term_label": "zinc ion binding",
  "gene_symbol": "CHORDC1",
  "gene_name": "Cysteine and histidine-rich domain-containing protein 1",
  "gene": "UniProtKB:Q9UHD1"
}